{
  "term_label": "Unknown cellular component",
  "gene_symbol": "PDE8B",
  "gene_name": "High affinity cAMP-specific and IBMX-insensitive 3',5'-cyclic phosphodiesterase 8B",
  "term_id": "UNKNOWN:0003",
  "gene": "UniProtKB:O95263"
}